silicate transmembrane transporter activity [GO:0015115] (molecular function) Sources: GOC:ai Relationships: is_a GO:0022857; is part of silicic acid import across plasma membrane [GO:0015708] Definition: Enables the transfer of silicates from one side of a membrane to the other. Silicates are the salts of silicic acids, and are usually composed of silicon and oxygen (Si[x]O[y]), one or more metals, and possibly hydrogen. Types of silicate include unisilicates, metasilicates and hydrous silicates.